{
  "term_id": "UNKNOWN:0002",
  "term_label": "Unknown biological process",
  "gene": "UniProtKB:Q86WV1",
  "gene_name": "Src kinase-associated phosphoprotein 1",
  "gene_symbol": "SKAP1"
}